{
  "gene_symbol": "SHLD1",
  "term_id": "GO:0035861",
  "gene": "UniProtKB:Q8IYI0",
  "term_label": "site of double-strand break",
  "gene_name": "Shieldin complex subunit 1"
}